facioacoustic ganglion development [GO:1903375] (biological process) Also known as: acoustico-facial VII-VIII ganglion complex development, acousticofacial ganglion development, facio-acoustic VII-VIII ganglion complex development, facio-acoustic ganglion complex VII-VIII development, facio-acoustic ganglion development Relationships: is a type of cranial ganglion development [GO:0061550] References: PMID:18356247 Sources: GOC:PARL, GOC:TermGenie, GOC:bf, GOC:mat, GO_REF:0000094 Definition: The process whose specific outcome is the progression of an acoustico-facial VII-VIII ganglion complex over time, from its formation to the mature structure.